{
  "gene_name": "RUN and FYVE domain-containing protein 4",
  "term_label": "autophagosome",
  "gene": "UniProtKB:Q6ZNE9",
  "gene_symbol": "RUFY4",
  "term_id": "GO:0005776"
}